{
  "gene": "UniProtKB:Q8IXQ9",
  "gene_symbol": "ETFBKMT",
  "gene_name": "Electron transfer flavoprotein beta subunit lysine methyltransferase",
  "term_id": "GO:0016279",
  "term_label": "protein-lysine N-methyltransferase activity"
}